{
  "gene_symbol": "NFKB2",
  "gene": "UniProtKB:Q00653",
  "term_label": "Unknown biological process",
  "gene_name": "Nuclear factor NF-kappa-B p100 subunit",
  "term_id": "UNKNOWN:0002"
}